{
  "gene_name": "Band 4.1-like protein 4B",
  "gene_symbol": "EPB41L4B",
  "term_id": "GO:0031032",
  "gene": "UniProtKB:Q9H329",
  "term_label": "actomyosin structure organization"
}